{
  "gene_name": "Destrin",
  "gene_symbol": "DSTN",
  "term_label": "actin filament severing",
  "term_id": "GO:0051014",
  "gene": "UniProtKB:P60981"
}